{
  "gene_name": "F-box only protein 50",
  "term_id": "GO:0019005",
  "gene_symbol": "NCCRP1",
  "term_label": "SCF ubiquitin ligase complex",
  "gene": "UniProtKB:Q6ZVX7"
}